D-serine ammonia-lyase activity [GO:0008721] (molecular function) Sources: EC:4.3.1.18 Relationships: is a type of ammonia-lyase activity [GO:0016841] Definition: Catalysis of the reaction: D-serine = pyruvate + NH3. Also known as: D-hydroxy amino acid dehydratase activity, D-hydroxyaminoacid dehydratase activity, D-serine ammonia-lyase (pyruvate-forming), D-serine deaminase activity, D-serine dehydrase activity, D-serine dehydratase (deaminating) activity, D-serine dehydratase activity, D-serine dehydration activity, D-serine hydro-lyase (deaminating) activity, D-serine hydrolase activity